hindbrain development [GO:0030902] (BP) Definition: The process whose specific outcome is the progression of the hindbrain over time, from its formation to the mature structure. The hindbrain is the posterior of the three primary divisions of the developing chordate brain, or the corresponding part of the adult brain (in vertebrates, includes the cerebellum, pons, and medulla oblongata and controls the autonomic functions and equilibrium). References: PMID:4975589, PMID:4992177 Also known as: rhombencephalon development Relationships: is a type of anatomical structure development [GO:0048856]; is part of brain development [GO:0007420]